regulation of endodermal cell fate specification [GO:0042663] (biological process) Also known as: regulation of endoderm cell fate specification Sources: GOC:go_curators Subtypes: GO:0042664 Relationships: is a type of regulation of cell fate specification [GO:0042659]; is a type of regulation of endodermal cell differentiation [GO:1903224]; regulates endodermal cell fate specification [GO:0001714] Definition: Any process that mediates the specification of a cell into an endoderm cell.